regulation of chondrocyte hypertrophy [GO:1903041] (biological process) References: PMID:23928032 Sources: GOC:TermGenie, GOC:mr, GO_REF:0000058 Subtypes: negative regulation of chondrocyte hypertrophy [GO:1903042], positive regulation of chondrocyte hypertrophy [GO:1903043] Definition: Any process that modulates the frequency, rate or extent of chondrocyte hypertrophy. Relationships: is a type of regulation of cell growth [GO:0001558]; is a type of regulation of developmental growth [GO:0048638]; is a type of regulation of chondrocyte development [GO:0061181]; regulates chondrocyte hypertrophy [GO:0003415]